{
  "term_label": "Unknown molecular function",
  "gene_symbol": "SLC37A3",
  "term_id": "UNKNOWN:0001",
  "gene_name": "Sugar phosphate exchanger 3",
  "gene": "UniProtKB:Q8NCC5"
}